{
  "gene": "UniProtKB:O60774",
  "gene_name": "Putative dimethylaniline monooxygenase [N-oxide-forming] 6",
  "term_id": "UNKNOWN:0003",
  "gene_symbol": "FMO6P",
  "term_label": "Unknown cellular component"
}